{
  "term_label": "Unknown molecular function",
  "gene": "UniProtKB:Q6UXD7",
  "gene_symbol": "SLC49A3",
  "gene_name": "Solute carrier family 49 member A3",
  "term_id": "UNKNOWN:0001"
}